{
  "gene_symbol": "ARHGAP25",
  "gene_name": "Rho GTPase-activating protein 25",
  "gene": "UniProtKB:P42331",
  "term_label": "phagocytic cup",
  "term_id": "GO:0001891"
}